{
  "gene_symbol": "GTF2A1",
  "term_id": "UNKNOWN:0001",
  "gene": "UniProtKB:P52655",
  "term_label": "Unknown molecular function",
  "gene_name": "Transcription initiation factor IIA subunit 1"
}